{
  "term_label": "2-oxoglutarate-dependent dioxygenase activity",
  "gene_symbol": "JMJD7",
  "gene_name": "Bifunctional peptidase and (3S)-lysyl hydroxylase JMJD7",
  "gene": "UniProtKB:P0C870",
  "term_id": "GO:0016706"
}